{
  "term_id": "UNKNOWN:0003",
  "gene": "UniProtKB:Q5H9L2",
  "term_label": "Unknown cellular component",
  "gene_symbol": "TCEAL5",
  "gene_name": "Transcription elongation factor A protein-like 5"
}